{
  "term_label": "Unknown molecular function",
  "term_id": "UNKNOWN:0001",
  "gene": "UniProtKB:Q6P0N0",
  "gene_name": "Mis18-binding protein 1",
  "gene_symbol": "MIS18BP1"
}